labrum development [GO:0048726] (biological process) Definition: The process whose specific outcome is the progression of the labrum over time, from its formation to the mature structure. Sources: GOC:rc Relationships: is a type of anatomical structure development [GO:0048856]; is part of clypeo-labral disc development [GO:0035213]